{
  "gene": "UniProtKB:Q9H9A7",
  "term_id": "UNKNOWN:0001",
  "gene_name": "RecQ-mediated genome instability protein 1",
  "term_label": "Unknown molecular function",
  "gene_symbol": "RMI1"
}